{
  "gene_symbol": "TMEM229A",
  "gene_name": "Transmembrane protein 229A",
  "gene": "UniProtKB:B2RXF0",
  "term_label": "Unknown cellular component",
  "term_id": "UNKNOWN:0003"
}